{
  "gene_name": "Fibrillin-3",
  "gene_symbol": "FBN3",
  "term_id": "GO:0042593",
  "gene": "UniProtKB:Q75N90",
  "term_label": "glucose homeostasis"
}